{
  "gene_symbol": "Q6ZRM9",
  "gene": "UniProtKB:Q6ZRM9",
  "term_label": "Unknown biological process",
  "gene_name": "Putative uncharacterized protein FLJ46235",
  "term_id": "UNKNOWN:0002"
}